glucose-6-phosphate transport [GO:0015760] (biological process) Definition: The directed movement of glucose-6-phosphate into, out of or within a cell, or between cells, by means of some agent such as a transporter or pore. Glucose-6-phosphate is a monophosphorylated derivative of glucose with the phosphate group attached to C-6. Sources: GOC:ai Relationships: is a type of GO:0015711; is a type of GO:0015712